{
  "gene_symbol": "ALG12",
  "term_label": "alpha-1,6-mannosyltransferase activity",
  "gene_name": "Dol-P-Man:Man(7)GlcNAc(2)-PP-Dol alpha-1,6-mannosyltransferase",
  "gene": "UniProtKB:Q9BV10",
  "term_id": "GO:0000009"
}